tyrosyl-DNA phosphodiesterase activity [GO:0070259] (MF) Definition: Catalysis of the hydrolysis of phosphotyrosyl groups formed as covalent intermediates (in DNA backbone breakage) between a DNA topoisomerase and DNA. Subtypes: 3'-tyrosyl-DNA phosphodiesterase activity [GO:0017005], 5'-tyrosyl-DNA phosphodiesterase activity [GO:0070260] References: PMID:16751265 Sources: GOC:elh Relationships: is a type of phosphoric diester hydrolase activity [GO:0008081]; is a type of catalytic activity, acting on DNA [GO:0140097] Note: See also the molecular function term 'DNA topoisomerase type I activity ; GO:0003917'.